regulation of macrophage activation [GO:0043030] (biological process) Definition: Any process that modulates the frequency or rate of macrophage activation. Subtypes: negative regulation of macrophage activation [GO:0043031], GO:0043032, regulation of microglial cell activation [GO:1903978] Sources: GOC:jl Relationships: is a type of regulation of leukocyte activation [GO:0002694]; regulates macrophage activation [GO:0042116] Also known as: regulation of macrophage polarization